choriogonadotropin hormone receptor activity [GO:0035472] (molecular function) Relationships: is a type of G protein-coupled receptor activity [GO:0004930]; is a type of protein-hormone receptor activity [GO:0016500]; has part choriogonadotropin hormone binding [GO:0038106] References: PMID:1922095 Sources: GOC:bf, ISBN:0198506732 Also known as: CG receptor activity, chorio-gonadotrophin receptor activity, chorionic gonadotropin hormone receptor Definition: Combining with the choriogonadotropin hormone to initiate a change in cell activity.